{
  "gene_name": "Prostate-specific antigen",
  "gene": "UniProtKB:P07288",
  "term_label": "extracellular space",
  "term_id": "GO:0005615",
  "gene_symbol": "KLK3"
}